L-arabinose 1-dehydrogenase (NADP+) activity [GO:0044103] (molecular function) References: PMID:16326697 Sources: GOC:jl Definition: Catalysis of the reaction: L-arabinose + NADP+ = L-arabinono-1,4-lactone + NADPH + H+. Relationships: is a type of GO:0016616